vascular endothelial growth factor receptor-2 signaling pathway [GO:0036324] (biological process) Also known as: FLK-1 signaling pathway, KDR signaling pathway, VEGFR-2 signaling pathway, VEGFR2 signaling pathway Definition: The series of molecular signals initiated by a ligand binding to a vascular endothelial growth factor receptor-2 (VEGFR-2) on the surface of a target cell, and ending with the regulation of a downstream cellular process, e.g. transcription. References: PMID:12967471 Sources: GOC:bf, GOC:uh, Wikipedia:Kinase_insert_domain_receptor, Wikipedia:VEGF_receptors Relationships: is a type of vascular endothelial growth factor receptor signaling pathway [GO:0048010]